{
  "gene_symbol": "HPS6",
  "gene_name": "BLOC-2 complex member HPS6",
  "term_id": "GO:0005765",
  "term_label": "lysosomal membrane",
  "gene": "UniProtKB:Q86YV9"
}